homoaconitate hydratase activity [GO:0004409] (molecular function) Definition: Catalysis of the reaction: (-)-homoisocitrate = cis-homoaconitate + H2O. Sources: EC:4.2.1.36, RHEA:15485 Also known as: (1R,2S)-1-hydroxybutane-1,2,4-tricarboxylate hydro-lyase [(Z)-but-1-ene-1,2,4-tricarboxylate-forming], 2-hydroxybutane-1,2,4-tricarboxylate hydro-lyase activity, HACN activity, Lys4, LysF, cis-homoaconitase activity, homoaconitase activity Relationships: is a type of hydro-lyase activity [GO:0016836]